{
  "term_label": "Unknown molecular function",
  "gene_name": "Uncharacterized protein C19orf47",
  "gene_symbol": "C19orf47",
  "term_id": "UNKNOWN:0001",
  "gene": "UniProtKB:Q8N9M1"
}